{
  "gene_symbol": "TERF1",
  "gene_name": "Telomeric repeat-binding factor 1",
  "term_id": "GO:0003720",
  "term_label": "telomerase activity",
  "gene": "UniProtKB:P54274"
}